{
  "gene": "UniProtKB:A0A0G2JLE6",
  "term_id": "UNKNOWN:0001",
  "gene_symbol": "KRTAP4-8",
  "gene_name": "HCG2042992",
  "term_label": "Unknown molecular function"
}